{
  "term_label": "regulation of transcription by RNA polymerase II",
  "gene": "UniProtKB:Q9C0D4",
  "gene_name": "Zinc finger protein 518B",
  "term_id": "GO:0006357",
  "gene_symbol": "ZNF518B"
}